{
  "gene_name": "Protein WWC2",
  "term_id": "GO:0046621",
  "gene_symbol": "WWC2",
  "gene": "UniProtKB:Q6AWC2",
  "term_label": "negative regulation of organ growth"
}